{
  "gene": "UniProtKB:Q9H7E9",
  "term_label": "Unknown molecular function",
  "term_id": "UNKNOWN:0001",
  "gene_name": "UPF0488 protein C8orf33",
  "gene_symbol": "C8orf33"
}